sulfate assimilation, phosphoadenylyl sulfate reduction by phosphoadenylyl-sulfate reductase (thioredoxin) [GO:0019379] (biological process) Relationships: is_a sulfate assimilation [GO:0000103]; BFO_0000051 GO:0004604 Sources: GOC:jl Definition: The pathway by which inorganic sulfate is processed and incorporated into sulfated compounds, where the phosphoadenylyl sulfate reduction step is catalyzed by the enzyme phosphoadenylyl-sulfate reductase (thioredoxin) (EC:1.8.4.8). Also known as: sulphate assimilation, phosphoadenylyl sulphate reduction by a phosphoadenylyl-sulphate reductase (thioredoxin)